aspartate 1-decarboxylase activity [GO:0004068] (MF) Definition: Catalysis of the reaction: L-aspartate = beta-alanine + CO2. Also known as: aspartic alpha-decarboxylase, L-aspartate 1-carboxy-lyase (beta-alanine-forming), L-aspartate 1-carboxy-lyase activity, L-aspartate alpha-decarboxylase activity, aspartate alpha-decarboxylase activity Note: Note that this term has a MetaCyc pathway reference as the pathway only has a single step. Relationships: is a type of carboxy-lyase activity [GO:0016831] Sources: EC:4.1.1.11